regulation of mitotic DNA replication initiation [GO:1903466] (BP) Relationships: is a type of regulation of DNA-templated DNA replication initiation [GO:0030174]; is a type of regulation of mitotic cell cycle DNA replication [GO:1903463]; regulates mitotic DNA replication initiation [GO:1902975] References: PMID:1234 Sources: GOC:TermGenie, GOC:mtg_cell_cycle, GO_REF:0000058 Also known as: regulation of DNA replication initiation involved in mitotic cell cycle DNA replication Definition: Any process that modulates the frequency, rate or extent of DNA replication initiation involved in mitotic DNA replication. Subtypes: regulation of mitotic DNA replication initiation from early origin [GO:0062212], regulation of mitotic DNA replication initiation from late origin [GO:0101017], negative regulation of mitotic DNA replication initiation [GO:1903467], positive regulation of DNA replication initiation [GO:1903468]